{
  "gene": "UniProtKB:Q9NZZ3",
  "term_label": "nuclear membrane reassembly",
  "gene_name": "Charged multivesicular body protein 5",
  "gene_symbol": "CHMP5",
  "term_id": "GO:0031468"
}